{
  "term_id": "GO:0000470",
  "gene": "UniProtKB:P56537",
  "gene_name": "Eukaryotic translation initiation factor 6",
  "gene_symbol": "EIF6",
  "term_label": "maturation of LSU-rRNA"
}